{
  "term_label": "cholesterol transfer activity",
  "term_id": "GO:0120020",
  "gene_name": "StAR-related lipid transfer protein 5",
  "gene": "UniProtKB:Q9NSY2",
  "gene_symbol": "STARD5"
}